{
  "term_label": "TRAPPII protein complex",
  "gene_symbol": "TRAPPC10",
  "gene": "UniProtKB:P48553",
  "term_id": "GO:1990071",
  "gene_name": "Trafficking protein particle complex subunit 10"
}